{
  "gene_symbol": "DNASE1L3",
  "gene_name": "Deoxyribonuclease gamma",
  "gene": "UniProtKB:Q13609",
  "term_label": "nucleus",
  "term_id": "GO:0005634"
}